beta-carotene isomerase activity [GO:0106365] (molecular function) Definition: Catalyzes the reaction: all-trans-beta-carotene = 9-cis-beta-carotene. References: PMID:19470589, PMID:22422982 Sources: RHEA:34455 Relationships: is a type of GO:0016859